{
  "gene_symbol": "EFNA5",
  "gene_name": "Ephrin-A5",
  "gene": "UniProtKB:P52803",
  "term_id": "GO:0022407",
  "term_label": "regulation of cell-cell adhesion"
}